carbon-sulfur lyase activity [GO:0016846] (molecular function) Definition: Catalysis of the elimination of hydrogen sulfide or substituted H2S. Relationships: is a type of lyase activity [GO:0016829] Subtypes: cystathionine gamma-lyase activity [GO:0004123], holocytochrome-c synthase activity [GO:0004408], lactoylglutathione lyase activity [GO:0004462], leukotriene-C4 synthase activity [GO:0004464], GO:0008826, selenocysteine lyase activity [GO:0009000], 1-aminocyclopropane-1-carboxylate synthase activity [GO:0016847], methionine gamma-lyase activity [GO:0018826], GO:0019148, sulfolactate sulfo-lyase activity [GO:0034010], L-cysteate sulfo-lyase activity [GO:0034011], S-ribosylhomocysteine lyase activity [GO:0043768], phosphosulfolactate synthase activity [GO:0043817], L-cystine L-cysteine-lyase (deaminating) [GO:0044540], S-adenosyl-L-methionine lyase activity [GO:0047625], GO:0047654, cysteine lyase activity [GO:0047803], cysteine-S-conjugate beta-lyase activity [GO:0047804], GO:0047869, homocysteine desulfhydrase activity [GO:0047982], L-3-cyanoalanine synthase activity [GO:0050017], 2-hydroxypropyl-CoM lyase activity [GO:0050555], S-(hydroxymethyl)glutathione synthase activity [GO:0051907], S-alkylthiohydroximate lyase activity [GO:0080108], L-cysteine desulfhydrase activity [GO:0080146], eoxin C4 synthase activity [GO:0097261], selenomethionine gamma-lyase activity [GO:0098600], GO:0098606, GO:0098607, hercynylcysteine sulfoxide lyase activity (ergothioneine-forming) [GO:1990411] Also known as: carbon-sulphur lyase activity Sources: EC:4.4.-.-